{
  "term_id": "GO:0004674",
  "gene_symbol": "CLK1",
  "term_label": "protein serine/threonine kinase activity",
  "gene": "UniProtKB:P49759",
  "gene_name": "Dual specificity protein kinase CLK1"
}